{
  "term_id": "GO:0003924",
  "gene_symbol": "RAB2B",
  "term_label": "GTPase activity",
  "gene": "UniProtKB:Q8WUD1",
  "gene_name": "Ras-related protein Rab-2B"
}